{
  "gene": "UniProtKB:Q96RV3",
  "term_id": "UNKNOWN:0002",
  "gene_name": "Pecanex-like protein 1",
  "gene_symbol": "PCNX1",
  "term_label": "Unknown biological process"
}